{
  "gene_name": "High affinity choline transporter 1",
  "term_label": "choline transport",
  "term_id": "GO:0015871",
  "gene_symbol": "SLC5A7",
  "gene": "UniProtKB:Q9GZV3"
}